{
  "gene": "UniProtKB:Q9H205",
  "term_id": "GO:0005886",
  "term_label": "plasma membrane",
  "gene_symbol": "OR2AG1",
  "gene_name": "Olfactory receptor 2AG1"
}